protein-N(PI)-phosphohistidine-cellobiose phosphotransferase system transporter activity [GO:0022874] (molecular function) Sources: GOC:mtg_transport, ISBN:0815340729 Also known as: cellobiose PTS transporter activity Relationships: is_a protein-N(PI)-phosphohistidine-sugar phosphotransferase activity [GO:0008982]; is a type of cellobiose transmembrane transporter activity [GO:0019191] Definition: Catalysis of the PEP-dependent, phosphoryl transfer-driven transport of substances across a membrane. The transport happens by catalysis of the reaction: protein N-phosphohistidine + cellobiose(out) = protein histidine + cellobiose phosphate(in). This differs from primary and secondary active transport in that the solute is modified during transport.